{
  "term_label": "striated muscle cell differentiation",
  "gene_symbol": "BVES",
  "gene_name": "Blood vessel epicardial substance",
  "gene": "UniProtKB:Q8NE79",
  "term_id": "GO:0051146"
}